{
  "term_id": "GO:0003723",
  "gene_name": "Histidine--tRNA ligase, mitochondrial",
  "gene": "UniProtKB:P49590",
  "gene_symbol": "HARS2",
  "term_label": "RNA binding"
}